interferon regulatory factor 3 complex [GO:0097072] (cellular component) Relationships: is a type of interferon regulatory factor complex [GO:0097071] References: PMID:12855817, PMID:14556004 Sources: GOC:cna Also known as: IRF3:IRF3 complex Definition: An interferon regulatory factor complex that consists of a homodimer of interferon regulatory factor 3.